brahma complex [GO:0035060] (cellular component) Definition: A SWI/SNF-type complex that contains 8 to 14 proteins, including both conserved (core) and nonconserved components; contains the ATPase product of the Drosophila brm (brahma) or mammalian SMARCA2/BAF190B/BRM gene, or an ortholog thereof. Relationships: is a type of SWI/SNF superfamily-type complex [GO:0070603] Also known as: BRM complex References: PMID:10809665, PMID:12482982 Sources: GOC:bhm